hexose catabolic process [GO:0019320] (biological process) Relationships: is a type of hexose metabolic process [GO:0019318]; is_a monosaccharide catabolic process [GO:0046365] Definition: The chemical reactions and pathways resulting in the breakdown of hexose, any monosaccharide with a chain of six carbon atoms in the molecule. Subtypes: fructose catabolic process [GO:0006001], glucose catabolic process [GO:0006007], rhamnose catabolic process [GO:0019301], mannose catabolic process [GO:0019309], GO:0019316, fucose catabolic process [GO:0019317], galactose catabolic process [GO:0019388], L-sorbose catabolic process [GO:0042850] Sources: ISBN:0198506732 Also known as: hexose breakdown, hexose catabolism, hexose degradation